{
  "term_label": "actin filament binding",
  "gene_symbol": "NEB",
  "gene_name": "Nebulin",
  "term_id": "GO:0051015",
  "gene": "UniProtKB:P20929"
}